response to phenylpropanoid [GO:0080184] (biological process) Relationships: is a type of GO:0042221 Sources: GOC:tb Subtypes: response to hydroxyisoflavone [GO:0033594], response to catechin [GO:1902168], cellular response to phenylpropanoid [GO:1905546] Definition: Any process that results in a change in state or activity of a cell or organism (in terms of movement, secretion, enzyme production, gene expression, etc.) as the result of a phenylpropanoid stimulus. The process begins with detection of the stimulus and ends with a change in state or activity or the cell or organism. A phenylpropanoid is any of secondary metabolites with structures based on a phenylpropane skeleton. The class includes phenylpropanoid esters, flavonoids, anthocyanins, coumarins and many small phenolic molecules. Phenylpropanoids are also precursors of lignin.